{
  "term_id": "GO:1990380",
  "gene": "UniProtKB:A8MYZ0",
  "gene_name": "Inactive ubiquitin carboxyl-terminal hydrolase MINDY-4B",
  "term_label": "K48-linked deubiquitinase activity",
  "gene_symbol": "MINDY4B"
}